posterior mesonephric tubule development [GO:0072166] (BP) Definition: The progression of the posterior mesonephric tubule over time, from its initial formation to the mature structure. The posterior mesonephric tubule is an epithelial tube that is part of the mesonephros. Sources: GOC:mtg_kidney_jan10 Relationships: is a type of mesonephric tubule development [GO:0072164]